{
  "term_id": "UNKNOWN:0002",
  "gene": "UniProtKB:Q9BZA5",
  "gene_name": "Putative gamma-taxilin 2",
  "term_label": "Unknown biological process",
  "gene_symbol": "TXLNGY"
}